regulation of protein localization to plasma membrane [GO:1903076] (biological process) Subtypes: GO:0042996, negative regulation of protein localization to plasma membrane [GO:1903077], positive regulation of protein localization to plasma membrane [GO:1903078], regulation of endosome to plasma membrane protein transport [GO:1905749], regulation of protein localization to prospore membrane [GO:2001231] Relationships: is a type of regulation of protein localization to cell periphery [GO:1904375]; is a type of regulation of protein localization to membrane [GO:1905475]; regulates protein localization to plasma membrane [GO:0072659] References: PMID:11602640 Sources: GOC:BHF, GOC:TermGenie, GOC:rl, GO_REF:0000058 Definition: Any process that modulates the frequency, rate or extent of protein localization to plasma membrane. Also known as: regulation of protein localization in plasma membrane, regulation of establishment of protein localisation in plasma membrane, regulation of establishment of protein localization in plasma membrane, regulation of establishment of protein localization to plasma membrane, regulation of protein localisation in plasma membrane, regulation of protein targeting to plasma membrane, regulation of protein-plasma membrane targeting